{
  "term_id": "GO:0034237",
  "gene_name": "A-kinase anchor protein 9",
  "term_label": "protein kinase A regulatory subunit binding",
  "gene": "UniProtKB:Q99996",
  "gene_symbol": "AKAP9"
}